{
  "gene_symbol": "LOC122526780",
  "gene": "UniProtKB:A0A590UJ96",
  "term_label": "Unknown molecular function",
  "term_id": "UNKNOWN:0001",
  "gene_name": "Uncharacterized protein"
}